FMN-binding domain binding [GO:0101016] (molecular function) Definition: Binding to the FMN-binding domain of a protein. References: PMID:15752726 Relationships: is a type of GO:0019904